{
  "term_id": "UNKNOWN:0002",
  "gene_symbol": "OR8U8",
  "gene": "UniProtKB:P0C7N1",
  "term_label": "Unknown biological process",
  "gene_name": "Olfactory receptor 8U8"
}